{
  "gene_symbol": "RNASE3",
  "gene": "UniProtKB:P12724",
  "term_label": "defense response to Gram-positive bacterium",
  "term_id": "GO:0050830",
  "gene_name": "Eosinophil cationic protein"
}